{
  "gene_symbol": "C17orf114",
  "term_label": "Unknown cellular component",
  "gene_name": "Uncharacterized protein C17orf114",
  "gene": "UniProtKB:A0A1B0GUV1",
  "term_id": "UNKNOWN:0003"
}